{
  "gene": "UniProtKB:Q9UPW8",
  "gene_symbol": "UNC13A",
  "term_id": "GO:0031594",
  "gene_name": "Protein unc-13 homolog A",
  "term_label": "neuromuscular junction"
}